{
  "term_id": "GO:0006508",
  "gene": "UniProtKB:Q8IVL8",
  "term_label": "proteolysis",
  "gene_symbol": "CPO",
  "gene_name": "Carboxypeptidase O"
}